{
  "gene_name": "Pygopus homolog 1",
  "gene": "UniProtKB:Q9Y3Y4",
  "gene_symbol": "PYGO1",
  "term_id": "UNKNOWN:0003",
  "term_label": "Unknown cellular component"
}